{
  "term_id": "GO:0005634",
  "gene_name": "Proline-rich protein PRCC",
  "gene": "UniProtKB:Q92733",
  "term_label": "nucleus",
  "gene_symbol": "PRCC"
}